{
  "gene": "UniProtKB:Q9H9F9",
  "term_label": "regulation of DNA-templated transcription",
  "term_id": "GO:0006355",
  "gene_symbol": "ACTR5",
  "gene_name": "Actin-related protein 5"
}